{
  "gene_name": "Sphingosine-1-phosphate lyase 1",
  "term_id": "GO:0030149",
  "term_label": "sphingolipid catabolic process",
  "gene": "UniProtKB:O95470",
  "gene_symbol": "SGPL1"
}